stereocilium bundle organization [GO:0160194] (biological process) Definition: A process that is carried out at the cellular level which results in the assembly, arrangement of constituent parts, or disassembly of a sensory hair cell stereocilium bundle. References: PMID:28266911, PMID:6978627 Relationships: is a type of GO:0016043